{
  "gene_name": "Radial spoke head protein 9 homolog",
  "gene_symbol": "RSPH9",
  "gene": "UniProtKB:Q9H1X1",
  "term_label": "axoneme assembly",
  "term_id": "GO:0035082"
}